{
  "gene_symbol": "NPY1R",
  "gene_name": "Neuropeptide Y receptor type 1",
  "term_id": "GO:0007218",
  "gene": "UniProtKB:P25929",
  "term_label": "neuropeptide signaling pathway"
}